{
  "gene_name": "Gastrin",
  "gene": "UniProtKB:P01350",
  "gene_symbol": "GAST",
  "term_id": "GO:0005615",
  "term_label": "extracellular space"
}